{
  "gene_name": "Proto-oncogene c-Rel",
  "gene_symbol": "REL",
  "term_id": "GO:0034097",
  "term_label": "response to cytokine",
  "gene": "UniProtKB:Q04864"
}